{
  "gene_symbol": "DEFA5",
  "term_label": "extracellular space",
  "gene": "UniProtKB:Q01523",
  "term_id": "GO:0005615",
  "gene_name": "Defensin alpha 5"
}